{
  "gene_symbol": "MYOD1",
  "gene": "UniProtKB:P15172",
  "term_id": "GO:0006357",
  "gene_name": "Myoblast determination protein 1",
  "term_label": "regulation of transcription by RNA polymerase II"
}